carbon catabolite regulation of transcription [GO:0045990] (biological process) Subtypes: carbon catabolite regulation of transcription from RNA polymerase II promoter [GO:0000429], GO:0045013, carbon catabolite activation of transcription [GO:0045991] Definition: A transcription regulation process in which the presence of one carbon source leads to the modulation of the frequency, rate, or extent of transcription of specific genes involved in the metabolism of other carbon sources. Relationships: is_a regulation of DNA-templated transcription [GO:0006355]; is_a cellular response to nutrient [GO:0031670] References: PMID:18359269, PMID:9618445 Sources: GOC:go_curators, GOC:mah Also known as: regulation of transcription by carbon catabolites